protein localization to T-tubule [GO:0036371] (biological process) Definition: A process in which a protein is transported to, or maintained in, the T-tubule. The T-tubule is an invagination of the plasma membrane of a muscle cell that extends inward from the cell surface around each myofibril. Relationships: is a type of GO:0072659 References: PMID:16292983 Sources: GOC:BHF, GOC:rl Also known as: protein localisation to T-tubule, protein localization to T tubule, protein localization to transverse tubule